{
  "term_id": "UNKNOWN:0001",
  "gene": "UniProtKB:Q15170",
  "term_label": "Unknown molecular function",
  "gene_symbol": "TCEAL1",
  "gene_name": "Transcription elongation factor A protein-like 1"
}